negative regulation of tensidol A biosynthetic process [GO:1900708] (biological process) Sources: GOC:TermGenie, GOC:di Relationships: is a type of GO:0034249; is a type of negative regulation of small molecule metabolic process [GO:0062014]; is a type of GO:1900377; is a type of regulation of tensidol A biosynthetic process [GO:1900707]; negatively regulates GO:1900605 Also known as: down regulation of tensidol A anabolism, down regulation of tensidol A biosynthesis, down regulation of tensidol A biosynthetic process, down regulation of tensidol A formation, down regulation of tensidol A synthesis, down-regulation of tensidol A anabolism, down-regulation of tensidol A biosynthesis, down-regulation of tensidol A biosynthetic process, down-regulation of tensidol A formation, down-regulation of tensidol A synthesis, downregulation of tensidol A anabolism, downregulation of tensidol A biosynthesis, downregulation of tensidol A biosynthetic process, downregulation of tensidol A formation, downregulation of tensidol A synthesis, inhibition of tensidol A anabolism, inhibition of tensidol A biosynthesis, inhibition of tensidol A formation, inhibition of tensidol A synthesis, negative regulation of tensidol A anabolism, negative regulation of tensidol A biosynthesis, negative regulation of tensidol A formation, negative regulation of tensidol A synthesis, inhibition of tensidol A biosynthetic process Definition: Any process that stops, prevents or reduces the frequency, rate or extent of tensidol A biosynthetic process.